mRNA transcription [GO:0009299] (biological process) Sources: GOC:jl Also known as: mRNA biosynthesis, mRNA biosynthetic process, mRNA synthesis, cellular mRNA transcription Subtypes: mRNA transcription by RNA polymerase II [GO:0042789] Relationships: is_a DNA-templated transcription [GO:0006351]; is a type of mRNA metabolic process [GO:0016071] Definition: The cellular synthesis of messenger RNA (mRNA) from a DNA template.